{
  "term_id": "UNKNOWN:0002",
  "gene_symbol": "SPACA7",
  "gene_name": "Sperm acrosome-associated protein 7",
  "term_label": "Unknown biological process",
  "gene": "UniProtKB:Q96KW9"
}